food vacuole [GO:0020020] (cellular component) Definition: Vacuole within a parasite used for digestion of the host cell cytoplasm. An example of this component is found in the Apicomplexa. Sources: GOC:mb Also known as: digestive vacuole Relationships: is a type of GO:0032010